{
  "gene_symbol": "ETV1",
  "term_id": "GO:0005634",
  "gene": "UniProtKB:P50549",
  "gene_name": "ETS translocation variant 1",
  "term_label": "nucleus"
}